{
  "gene": "UniProtKB:Q9BYQ9",
  "gene_name": "Keratin-associated protein 4-8",
  "term_id": "UNKNOWN:0003",
  "term_label": "Unknown cellular component",
  "gene_symbol": "KRTAP4-8"
}